{
  "gene_symbol": "ZNF500",
  "term_label": "Unknown cellular component",
  "gene": "UniProtKB:O60304",
  "term_id": "UNKNOWN:0003",
  "gene_name": "Zinc finger protein 500"
}